complement component C5a receptor activity [GO:0004878] (molecular function) Also known as: C5a anaphylatoxin receptor activity Relationships: is a type of GO:0001847; is_a complement receptor activity [GO:0004875]; is part of GO:0038178; has part complement component C5a binding [GO:0001856] Sources: GOC:add, GOC:mah, GOC:pg, GOC:signaling, ISBN:0781735149 Definition: Combining with the C5a product of the complement cascade and transmitting the signal from one side of the membrane to the other to initiate a change in cell activity.